{
  "term_id": "GO:0004126",
  "gene_name": "DNA dC-dU-editing enzyme APOBEC-3G",
  "gene": "UniProtKB:Q9HC16",
  "gene_symbol": "APOBEC3G",
  "term_label": "cytidine deaminase activity"
}